negative regulation of protein activation cascade [GO:2000258] (biological process) Also known as: negative regulation of protein activation pathway, negative regulation of protein activitory cascade Definition: Any process that stops, prevents or reduces the frequency, rate or extent of protein activation cascade. Subtypes: GO:0002257, negative regulation of Toll receptor ligand protein activation cascade [GO:0160035], negative regulation of blood coagulation, common pathway [GO:2000261], GO:2000264, negative regulation of blood coagulation, intrinsic pathway [GO:2000267] Sources: GOC:mah Relationships: is a type of negative regulation of protein maturation [GO:1903318]; is a type of regulation of protein activation cascade [GO:2000257]; negatively regulates protein activation cascade [GO:0072376]